{
  "gene": "UniProtKB:P30876",
  "gene_name": "DNA-directed RNA polymerase II subunit RPB2",
  "gene_symbol": "POLR2B",
  "term_id": "GO:0006354",
  "term_label": "DNA-templated transcription elongation"
}